{
  "gene_symbol": "PAXIP1",
  "term_id": "GO:0060261",
  "term_label": "positive regulation of transcription initiation by RNA polymerase II",
  "gene": "UniProtKB:Q6ZW49",
  "gene_name": "PAX-interacting protein 1"
}